{
  "gene_symbol": "KDM7A",
  "term_id": "GO:0006338",
  "gene_name": "Lysine-specific demethylase 7A",
  "term_label": "chromatin remodeling",
  "gene": "UniProtKB:Q6ZMT4"
}